{
  "term_label": "protein serine/threonine phosphatase inhibitor activity",
  "gene": "UniProtKB:Q8TAE6",
  "gene_name": "Protein phosphatase 1 regulatory subunit 14C",
  "term_id": "GO:0004865",
  "gene_symbol": "PPP1R14C"
}